{
  "gene_symbol": "NOPCHAP1",
  "gene_name": "NOP protein chaperone 1",
  "gene": "UniProtKB:Q8N5I9",
  "term_label": "box C/D snoRNP assembly",
  "term_id": "GO:0000492"
}